{
  "term_label": "poly(ADP-ribose) glycohydrolase activity",
  "gene_symbol": "ADPRS",
  "gene": "UniProtKB:Q9NX46",
  "term_id": "GO:0004649",
  "gene_name": "ADP-ribosylhydrolase ARH3"
}